{
  "gene_symbol": "ADORA2B",
  "term_label": "vasodilation",
  "gene_name": "Adenosine receptor A2b",
  "term_id": "GO:0042311",
  "gene": "UniProtKB:P29275"
}